{
  "term_label": "Unknown molecular function",
  "term_id": "UNKNOWN:0001",
  "gene_name": "S-acyl fatty acid synthase thioesterase, medium chain",
  "gene": "UniProtKB:Q9NV23",
  "gene_symbol": "OLAH"
}